{
  "gene_symbol": "ZNF414",
  "term_id": "UNKNOWN:0002",
  "term_label": "Unknown biological process",
  "gene_name": "Zinc finger protein 414",
  "gene": "UniProtKB:Q96IQ9"
}